Gemin3-Gemin4-Gemin5 complex [GO:0034716] (cellular component) Relationships: is a type of intracellular protein-containing complex [GO:0140535] References: PMID:17640873 Sources: GOC:mah Definition: A protein complex that contains Gemin3 (DDX20), Gemin4, and Gemin5, and can bind to snRNAs; may be an intermediate in SMN complex assembly.